convergent extension involved in organogenesis [GO:0060029] (biological process) References: PMID:12062082 Sources: GOC:dph Subtypes: convergent extension involved in neural plate elongation [GO:0022007], convergent extension involved in nephron morphogenesis [GO:0072045], GO:0090253, convergent extension involved in rhombomere morphogenesis [GO:1904125], convergent extension involved in notochord morphogenesis [GO:1904126] Definition: The morphogenetic process in which an epithelium narrows along one axis and lengthens in a perpendicular axis contribution to the shaping of an organ. Relationships: is_a convergent extension [GO:0060026]; is part of animal organ development [GO:0048513]